{
  "gene_symbol": "SCN4B",
  "gene_name": "Sodium channel subunit beta-4",
  "term_label": "membrane depolarization during cardiac muscle cell action potential",
  "gene": "UniProtKB:Q8IWT1",
  "term_id": "GO:0086012"
}